{
  "gene": "UniProtKB:P01275",
  "term_id": "GO:0043066",
  "term_label": "negative regulation of apoptotic process",
  "gene_name": "Pro-glucagon",
  "gene_symbol": "GCG"
}